2-dehydro-3-deoxy-phosphogluconate aldolase activity [GO:0008675] (molecular function) Definition: Catalysis of the reaction: 2-dehydro-3-deoxy-D-gluconate 6-phosphate = pyruvate + D-glyceraldehyde 3-phosphate. Sources: EC:4.1.2.14 Also known as: 2-dehydro-3-deoxy-D-gluconate-6-phosphate D-glyceraldehyde-3-phosphate-lyase (pyruvate-forming), 2-dehydro-3-deoxy-D-gluconate-6-phosphate D-glyceraldehyde-3-phosphate-lyase activity, 2-keto-3-deoxy-6-phosphogluconate aldolase activity, 2-keto-3-deoxy-6-phosphogluconic aldolase activity, 2-keto-3-deoxygluconate-6-P-aldolase activity, 2-keto-3-deoxygluconate-6-phosphate aldolase activity, 2-oxo-3-deoxy-6-phosphogluconate aldolase activity, 6-phospho-2-keto-3-deoxygluconate aldolase activity, KDPG aldolase activity, KDPG-aldolase activity, ODPG aldolase activity, phospho-2-dehydro-3-deoxygluconate aldolase activity, phospho-2-keto-3-deoxygluconate aldolase activity, phospho-2-keto-3-deoxygluconic aldolase activity Relationships: is a type of aldehyde-lyase activity [GO:0016832]